{
  "term_id": "GO:0070527",
  "gene_name": "Tyrosine-protein kinase receptor TYRO3",
  "term_label": "platelet aggregation",
  "gene_symbol": "TYRO3",
  "gene": "UniProtKB:Q06418"
}